{
  "term_id": "GO:0045893",
  "gene_symbol": "MSANTD1",
  "gene": "UniProtKB:Q6ZTZ1",
  "term_label": "positive regulation of DNA-templated transcription",
  "gene_name": "Myb_SANT-like DNA-binding domain-containing protein 1"
}